{
  "gene_name": "Speedy protein E2B",
  "gene": "UniProtKB:A6NHP3",
  "term_label": "protein kinase binding",
  "term_id": "GO:0019901",
  "gene_symbol": "SPDYE2B"
}